{
  "gene": "UniProtKB:Q13554",
  "term_id": "GO:0014069",
  "term_label": "postsynaptic density",
  "gene_symbol": "CAMK2B",
  "gene_name": "Calcium_calmodulin-dependent protein kinase type II subunit beta"
}